methylmalonyl-CoA carboxytransferase activity [GO:0047154] (molecular function) Relationships: is a type of carboxyl- or carbamoyltransferase activity [GO:0016743] Sources: EC:2.1.3.1, MetaCyc:2.1.3.1-RXN Also known as: methylmalonyl-CoA carboxyltransferase activity, (S)-2-methyl-3-oxopropanoyl-CoA:pyruvate, (S)-2-methyl-3-oxopropanoyl-CoA:pyruvate carboxyltransferase activity, (S)-methylmalonyl-CoA:pyruvate carboxyltransferase activity, (S)-methylmalonyl-CoA:pyruvate carboxytransferase activity, methylmalonyl coenzyme A carboxyltransferase activity, methylmalonyl-CoA transcarboxylase activity, oxalacetic transcarboxylase activity, transcarboxylase activity Definition: Catalysis of the reaction: pyruvate + D-methylmalonyl-CoA = oxaloacetic acid + propionyl-CoA.